negative regulation of actin filament binding [GO:1904530] (biological process) Relationships: is a type of negative regulation of protein binding [GO:0032091]; negatively regulates actin filament binding [GO:0051015] Definition: Any process that stops, prevents or reduces the frequency, rate or extent of actin filament binding. References: PMID:24520051 Sources: GOC:TermGenie, GOC:als, GO_REF:0000059 Also known as: down regulation of F-actin binding, down regulation of actin filament binding, down-regulation of F-actin binding, down-regulation of actin filament binding, downregulation of F-actin binding, downregulation of actin filament binding, negative regulation of F-actin binding, inhibition of F-actin binding, inhibition of actin filament binding, down regulation of actin cross-linking activity, down-regulation of actin cross-linking activity, downregulation of actin cross-linking activity, inhibition of actin cross-linking activity, negative regulation of actin cross-linking activity